response to cyclodiene [GO:0046682] (biological process) Also known as: cyclodiene resistance, cyclodiene susceptibility/resistance Sources: ISBN:0877797099 Relationships: is a type of response to insecticide [GO:0017085] Definition: Any process that results in a change in state or activity of a cell or an organism (in terms of movement, secretion, enzyme production, gene expression, etc.) as a result of a cyclodiene stimulus. A cyclodiene is any organic insecticide (as dieldrin or chlordane) with a chlorinated methylene group forming a bridge across a 6-membered carbon ring.